{
  "term_label": "cytosol",
  "gene_symbol": "NT5C1B",
  "term_id": "GO:0005829",
  "gene": "UniProtKB:Q96P26",
  "gene_name": "Cytosolic 5'-nucleotidase 1B"
}